{
  "gene_name": "Prostaglandin E2 receptor EP1 subtype",
  "term_id": "GO:0006954",
  "gene": "UniProtKB:P34995",
  "term_label": "inflammatory response",
  "gene_symbol": "PTGER1"
}